undecaprenol kinase activity [GO:0009038] (molecular function) Subtypes: all-trans undecaprenol kinase activity [GO:0036432], di-trans, poly-cis-undecaprenol kinase activity [GO:0036433] Also known as: isoprenoid alcohol kinase (phosphorylating), isoprenoid alcohol kinase activity, isoprenoid alcohol phosphokinase activity, isoprenoid-alcohol kinase activity, polyisoprenol kinase activity, ATP:undecaprenol phosphotransferase activity, C55-isoprenoid alcohol kinase activity, C55-isoprenoid alcohol phosphokinase activity, C55-isoprenyl alcohol phosphokinase activity Relationships: is_a kinase activity [GO:0016301]; is a type of GO:0016773 Definition: Catalysis of the reaction: ATP + undecaprenol = ADP + undecaprenyl phosphate. Sources: GOC:curators